regulation of syringal lignin catabolic process [GO:1901469] (biological process) Relationships: is a type of regulation of catabolic process [GO:0009894]; is a type of GO:2000762; regulates syringal lignin catabolic process [GO:1901065] Definition: Any process that modulates the frequency, rate or extent of syringal lignin catabolic process. Subtypes: negative regulation of syringal lignin catabolic process [GO:1901470], positive regulation of syringal lignin catabolic process [GO:1901471] Sources: GOC:TermGenie, GOC:mengo_curators Also known as: regulation of S-lignin catabolic process, regulation of syringal lignin breakdown, regulation of syringal lignin catabolism, regulation of syringal lignin degradation